{
  "term_label": "sodium:proton antiporter activity",
  "gene_symbol": "SLC9A8",
  "gene": "UniProtKB:Q9Y2E8",
  "term_id": "GO:0015385",
  "gene_name": "Sodium_hydrogen exchanger 8"
}